{
  "gene": "UniProtKB:P25054",
  "gene_symbol": "APC",
  "gene_name": "Adenomatous polyposis coli protein",
  "term_label": "cytoplasmic microtubule",
  "term_id": "GO:0005881"
}